positive regulation of pupariation [GO:0106025] (biological process) Sources: GOC:hjd Relationships: is a type of positive regulation of multicellular organismal process [GO:0051240]; is a type of regulation of pupariation [GO:0106023]; positively regulates pupariation [GO:0035073] Definition: Any process that activates or increases the frequency, rate or extent of onset of pupariation.